{
  "term_id": "GO:0005634",
  "gene_name": "Zinc finger protein 282",
  "gene": "UniProtKB:Q9UDV7",
  "gene_symbol": "ZNF282",
  "term_label": "nucleus"
}